{
  "term_id": "GO:0006355",
  "gene_name": "Zinc finger protein 724",
  "gene": "UniProtKB:A8MTY0",
  "term_label": "regulation of DNA-templated transcription",
  "gene_symbol": "ZNF724"
}